{
  "term_label": "desensitization of G protein-coupled receptor signaling pathway",
  "term_id": "GO:0002029",
  "gene": "UniProtKB:P25098",
  "gene_name": "Beta-adrenergic receptor kinase 1",
  "gene_symbol": "GRK2"
}